wobble position cytosine ribose methylation [GO:0002131] (BP) Sources: GOC:hjd, ISBN:155581073X Definition: The process in which the ribose of cytidine at position 34 in the anticodon of a tRNA is post-transcriptionally methylated at the 2'-O position. Relationships: is a type of wobble position ribose methylation [GO:0002130]